{
  "term_label": "potassium ion leak channel activity",
  "gene_symbol": "KCNK1",
  "term_id": "GO:0022841",
  "gene_name": "Potassium channel subfamily K member 1",
  "gene": "UniProtKB:O00180"
}